{
  "term_id": "GO:0043625",
  "term_label": "delta DNA polymerase complex",
  "gene": "UniProtKB:P28340",
  "gene_symbol": "POLD1",
  "gene_name": "DNA polymerase delta catalytic subunit"
}